{
  "gene_symbol": "PCDHGC3",
  "term_label": "plasma membrane",
  "term_id": "GO:0005886",
  "gene": "UniProtKB:Q9UN70",
  "gene_name": "Protocadherin gamma-C3"
}